histidine phosphotransfer kinase activity [GO:0009927] (molecular function) Relationships: is a type of protein kinase activity [GO:0004672]; is a type of GO:0060089 References: PMID:11842140, PMID:31386843 Definition: Serves as a phospho-His intermediate enabling the transfer of phospho group between a hybrid kinase and a response regulator.